terminal bouton [GO:0043195] (CC) Definition: Terminal inflated portion of the axon, containing the specialized apparatus necessary to release neurotransmitters. The axon terminus is considered to be the whole region of thickening and the terminal bouton is a specialized region of it. References: PMID:10218156, PMID:8409967 Sources: GOC:dph, GOC:mc, GOC:nln Also known as: bouton, presynaptic bouton, synaptic bouton, terminal button Relationships: is a type of presynapse [GO:0098793]; is part of axon terminus [GO:0043679] Subtypes: type I terminal bouton [GO:0061174], GO:0061175, type III terminal bouton [GO:0097467], multiple synapse bouton [GO:0150086], C bouton [GO:1990024], F bouton [GO:1990025], GO:1990026, S bouton [GO:1990027], rod bipolar cell terminal bouton [GO:1990795], photoreceptor cell terminal bouton [GO:1990796]